{
  "term_id": "GO:0031966",
  "gene_name": "Cytochrome c oxidase subunit 7A2, mitochondrial",
  "gene_symbol": "COX7A2",
  "gene": "UniProtKB:P14406",
  "term_label": "mitochondrial membrane"
}